{
  "gene_symbol": "NANOS2",
  "gene": "UniProtKB:P60321",
  "gene_name": "Nanos homolog 2",
  "term_id": "GO:0048477",
  "term_label": "oogenesis"
}